positive regulation of midbrain dopaminergic neuron differentiation [GO:1904958] (BP) References: PMID:21347250 Sources: GOC:PARL, GOC:TermGenie, GOC:bf, GO_REF:0000058 Also known as: positive regulation of DA neurogenesis from midbrain floor plate, positive regulation of mDA neuron differentiation, positive regulation of midbrain DA neurogenesis, positive regulation of midbrain dopaminergic neuron production, up regulation of DA neurogenesis from midbrain floor plate, up regulation of mDA neuron differentiation, up regulation of midbrain DA neurogenesis, up regulation of midbrain dopaminergic neuron differentiation, up regulation of midbrain dopaminergic neuron production, up-regulation of DA neurogenesis from midbrain floor plate, up-regulation of mDA neuron differentiation, up-regulation of midbrain DA neurogenesis, up-regulation of midbrain dopaminergic neuron differentiation, up-regulation of midbrain dopaminergic neuron production, upregulation of DA neurogenesis from midbrain floor plate, upregulation of mDA neuron differentiation, upregulation of midbrain DA neurogenesis, upregulation of midbrain dopaminergic neuron differentiation, upregulation of midbrain dopaminergic neuron production, activation of DA neurogenesis from midbrain floor plate, activation of mDA neuron differentiation, activation of midbrain DA neurogenesis, activation of midbrain dopaminergic neuron differentiation, activation of midbrain dopaminergic neuron production Relationships: is a type of positive regulation of dopaminergic neuron differentiation [GO:1904340]; is a type of regulation of midbrain dopaminergic neuron differentiation [GO:1904956]; positively regulates midbrain dopaminergic neuron differentiation [GO:1904948] Definition: Any process that activates or increases the frequency, rate or extent of midbrain dopaminergic neuron differentiation.